{
  "gene": "UniProtKB:Q9NPP4",
  "gene_symbol": "NLRC4",
  "term_label": "defense response to bacterium",
  "gene_name": "NLR family CARD domain-containing protein 4",
  "term_id": "GO:0042742"
}